{
  "term_label": "positive regulation of transcription by RNA polymerase II",
  "gene_symbol": "SMARCA4",
  "gene_name": "Transcription activator BRG1",
  "term_id": "GO:0045944",
  "gene": "UniProtKB:P51532"
}